rRNA (cytosine-C5-)-methyltransferase activity [GO:0009383] (molecular function) Relationships: is_a C-methyltransferase activity [GO:0008169]; is a type of GO:0016434 References: PMID:10026269, PMID:18786544 Sources: GOC:imk Definition: Catalysis of the transfer of a methyl group from S-adenosyl-L-methionine to cytosine to form 5-methylcytosine in small subunit ribosomal RNA. Also known as: rRNA (cytosine-C5-967)-methyltransferase activity, rRNA m5C967 methyltransferase activity